{
  "term_label": "plasma membrane",
  "gene_symbol": "OR51H1",
  "gene": "UniProtKB:Q8NH63",
  "term_id": "GO:0005886",
  "gene_name": "Olfactory receptor 51H1"
}